{
  "term_id": "GO:0048278",
  "gene_symbol": "STX12",
  "gene": "UniProtKB:Q86Y82",
  "gene_name": "Syntaxin-12",
  "term_label": "vesicle docking"
}